{
  "gene": "UniProtKB:Q9Y4K3",
  "term_id": "GO:0005737",
  "gene_symbol": "TRAF6",
  "gene_name": "TNF receptor-associated factor 6",
  "term_label": "cytoplasm"
}